{
  "term_id": "GO:0008053",
  "gene_name": "Bcl-2-related protein A1",
  "gene_symbol": "BCL2A1",
  "term_label": "mitochondrial fusion",
  "gene": "UniProtKB:Q16548"
}